{
  "gene_name": "2-hydroxyacyl-CoA lyase 2",
  "gene": "UniProtKB:A1L0T0",
  "term_label": "isoleucine biosynthetic process",
  "term_id": "GO:0009097",
  "gene_symbol": "ILVBL"
}